positive regulation of lymphocyte activation [GO:0051251] (biological process) Definition: Any process that activates or increases the frequency, rate or extent of lymphocyte activation. Subtypes: lymphocyte costimulation [GO:0031294], positive regulation of natural killer cell activation [GO:0032816], positive regulation of lymphocyte differentiation [GO:0045621], positive regulation of lymphocyte proliferation [GO:0050671], positive regulation of T cell activation [GO:0050870], GO:0050871 Also known as: up regulation of lymphocyte activation, up-regulation of lymphocyte activation, upregulation of lymphocyte activation, activation of lymphocyte activation, stimulation of lymphocyte activation Relationships: is a type of positive regulation of leukocyte activation [GO:0002696]; is a type of GO:0051249; positively regulates lymphocyte activation [GO:0046649] Sources: GOC:ai